{
  "term_label": "plasma membrane",
  "term_id": "GO:0005886",
  "gene": "UniProtKB:Q9UQ05",
  "gene_name": "Potassium voltage-gated channel subfamily H member 4",
  "gene_symbol": "KCNH4"
}